{
  "gene_name": "Actin, alpha skeletal muscle",
  "gene_symbol": "ACTA1",
  "term_label": "stress fiber",
  "gene": "UniProtKB:P68133",
  "term_id": "GO:0001725"
}